{
  "gene": "UniProtKB:Q9BXV9",
  "term_label": "Unknown biological process",
  "term_id": "UNKNOWN:0002",
  "gene_symbol": "GON7",
  "gene_name": "EKC_KEOPS complex subunit GON7"
}